{
  "term_id": "GO:0015746",
  "term_label": "citrate transport",
  "gene_name": "Na(+)_dicarboxylate cotransporter 3",
  "gene": "UniProtKB:Q8WWT9",
  "gene_symbol": "SLC13A3"
}